positive regulation of exo-alpha-sialidase activity [GO:1903017] (biological process) Relationships: is a type of positive regulation of hydrolase activity [GO:0051345]; positively regulates exo-alpha-sialidase activity [GO:0004308] Note: human serum amyloid P component (SAP) P02743 inhibits viral neuraminidase, NA (exo-alpha-sialidase activity) demonstrated in Figure 4A PMID:23544079, (IDA) Also known as: positive regulation of N-acylneuraminate glycohydrolase activity, positive regulation of acetylneuraminidase activity, positive regulation of acetylneuraminyl hydrolase activity, positive regulation of alpha-neuraminidase activity, positive regulation of neuraminidase activity, positive regulation of sialidase activity, up regulation of N-acylneuraminate glycohydrolase activity, up regulation of acetylneuraminidase activity, up regulation of acetylneuraminyl hydrolase activity, up regulation of alpha-neuraminidase activity, up regulation of exo-alpha-sialidase activity, up regulation of neuraminidase activity, up regulation of sialidase activity, up-regulation of N-acylneuraminate glycohydrolase activity, up-regulation of acetylneuraminidase activity, up-regulation of acetylneuraminyl hydrolase activity, up-regulation of alpha-neuraminidase activity, up-regulation of exo-alpha-sialidase activity, up-regulation of neuraminidase activity, up-regulation of sialidase activity, upregulation of N-acylneuraminate glycohydrolase activity, upregulation of acetylneuraminidase activity, upregulation of acetylneuraminyl hydrolase activity, upregulation of alpha-neuraminidase activity, upregulation of exo-alpha-sialidase activity, upregulation of neuraminidase activity, upregulation of sialidase activity, activation of N-acylneuraminate glycohydrolase activity, activation of acetylneuraminidase activity, activation of acetylneuraminyl hydrolase activity, activation of alpha-neuraminidase activity, activation of exo-alpha-sialidase activity, activation of neuraminidase activity, activation of sialidase activity References: PMID:23544079 Sources: GOC:BHF, GOC:TermGenie, GOC:rl, GO_REF:0000059 Definition: Any process that activates or increases the frequency, rate or extent of exo-alpha-sialidase activity.